{
  "term_id": "UNKNOWN:0002",
  "gene_name": "Neuronal migration protein doublecortin",
  "gene": "UniProtKB:O43602",
  "gene_symbol": "DCX",
  "term_label": "Unknown biological process"
}